G protein-coupled amine receptor activity [GO:0008227] (molecular function) Also known as: G-protein coupled amine receptor activity, amine receptor activity, G-protein coupled, biogenic amine receptor Definition: Combining with an extracellular amine and transmitting the signal across the membrane by activating an associated G-protein; promotes the exchange of GDP for GTP on the alpha subunit of a heterotrimeric G-protein complex. Sources: GOC:bf, GOC:dph Relationships: is_a GO:0004930 Subtypes: GO:0001594, adrenergic receptor activity [GO:0004935], histamine receptor activity [GO:0004969], octopamine receptor activity [GO:0004989], G protein-coupled serotonin receptor activity [GO:0004993], tyramine receptor activity [GO:0008226], GO:0016907, 2-phenylethylamine receptor activity [GO:1990080]